{
  "term_label": "calcium channel activity",
  "gene": "UniProtKB:Q9UI40",
  "gene_name": "Sodium_potassium_calcium exchanger 2",
  "gene_symbol": "SLC24A2",
  "term_id": "GO:0005262"
}